{
  "gene": "UniProtKB:Q9HAT8",
  "term_label": "protein polyubiquitination",
  "term_id": "GO:0000209",
  "gene_name": "E3 ubiquitin-protein ligase pellino homolog 2",
  "gene_symbol": "PELI2"
}